{
  "term_label": "Unknown molecular function",
  "gene_name": "CDK5 and ABL1 enzyme substrate 2",
  "gene": "UniProtKB:Q9BTV7",
  "gene_symbol": "CABLES2",
  "term_id": "UNKNOWN:0001"
}